dorsal/ventral pattern formation [GO:0009953] (BP) Relationships: is_a regionalization [GO:0003002] Sources: GOC:dph, GOC:go_curators, GOC:isa_complete, GOC:tb Subtypes: dorsal/ventral pattern formation, imaginal disc [GO:0007450], spinal cord dorsal/ventral patterning [GO:0021513], forebrain dorsal/ventral pattern formation [GO:0021798], GO:0021904, GO:0048263, determination of ventral identity [GO:0048264], embryonic heart tube dorsal/ventral pattern formation [GO:0060970] Definition: The regionalization process in which the areas along the dorsal/ventral axis are established that will lead to differences in cell differentiation. The dorsal/ventral axis is defined by a line that runs orthogonal to both the anterior/posterior and left/right axes. The dorsal end is defined by the upper or back side of an organism. The ventral end is defined by the lower or front side of an organism. Also known as: dorsal-ventral pattern formation, dorsoventral pattern formation, dorsal/ventral pattern specification